{
  "gene_symbol": "MAPK7",
  "gene": "UniProtKB:Q13164",
  "gene_name": "Mitogen-activated protein kinase 7",
  "term_label": "cytoplasm",
  "term_id": "GO:0005737"
}